{
  "gene": "UniProtKB:Q9NYX4",
  "gene_name": "Neuron-specific vesicular protein calcyon",
  "gene_symbol": "CALY",
  "term_id": "GO:0016020",
  "term_label": "membrane"
}